{
  "gene_name": "Neuronal acetylcholine receptor subunit beta-2",
  "gene_symbol": "CHRNB2",
  "term_label": "acetylcholine-gated monoatomic cation-selective channel activity",
  "gene": "UniProtKB:P17787",
  "term_id": "GO:0022848"
}